{
  "term_id": "GO:0007420",
  "gene_symbol": "NOTO",
  "gene": "UniProtKB:A8MTQ0",
  "term_label": "brain development",
  "gene_name": "Homeobox protein notochord"
}